{
  "gene_name": "Cytoplasmic dynein 1 heavy chain 1",
  "gene": "UniProtKB:Q14204",
  "term_label": "cell cortex",
  "term_id": "GO:0005938",
  "gene_symbol": "DYNC1H1"
}